membrane raft organization [GO:0031579] (biological process) Definition: A process that is carried out at the cellular level which results in the assembly, arrangement of constituent parts, or disassembly of membrane rafts, small (10-200 nm), heterogeneous, highly dynamic, sterol- and sphingolipid-enriched membrane domains that compartmentalize cellular processes. Sources: GOC:dph, GOC:jl, GOC:mah Also known as: lipid raft organization, membrane raft organisation, membrane raft organization and biogenesis Relationships: is a type of GO:0061024 Subtypes: membrane raft assembly [GO:0001765], GO:0031580, GO:0044857